paraspeckles [GO:0042382] (cellular component) Definition: Discrete subnuclear bodies in the interchromatin nucleoplasmic space, often located adjacent to nuclear specks. 10-20 paraspeckles are typically found in human cell nuclei. Relationships: is a type of nuclear ribonucleoprotein granule [GO:0140168] References: PMID:11790299 Sources: GOC:jl